{
  "gene_symbol": "TSPAN31",
  "gene_name": "Tetraspanin-31",
  "term_label": "Unknown molecular function",
  "term_id": "UNKNOWN:0001",
  "gene": "UniProtKB:Q12999"
}